{
  "term_id": "GO:0004844",
  "gene_name": "G_T mismatch-specific thymine DNA glycosylase",
  "gene": "UniProtKB:Q13569",
  "gene_symbol": "TDG",
  "term_label": "uracil DNA N-glycosylase activity"
}